{
  "term_id": "GO:0017157",
  "gene": "UniProtKB:Q99719",
  "gene_symbol": "SEPTIN5",
  "gene_name": "Septin-5",
  "term_label": "regulation of exocytosis"
}